response to leptin [GO:0044321] (biological process) Definition: Any process that results in a change in state or activity of a cell or an organism (in terms of movement, secretion, enzyme production, gene expression, etc.) as a result of a leptin stimulus. Leptin is a hormone manufactured primarily in the adipocytes of white adipose tissue, and the level of circulating leptin is directly proportional to the total amount of fat in the body. It plays a key role in regulating energy intake and energy expenditure, including appetite and metabolism]. Sources: GOC:yaf Also known as: response to leptin stimulus Relationships: is a type of GO:0009725 Subtypes: cellular response to leptin stimulus [GO:0044320]